{
  "gene_symbol": "NBEAL2",
  "gene": "UniProtKB:Q6ZNJ1",
  "gene_name": "Neurobeachin-like protein 2",
  "term_id": "GO:0005829",
  "term_label": "cytosol"
}